blood microparticle [GO:0072562] (cellular component) Definition: A phospholipid microvesicle that is derived from any of several cell types, such as platelets, blood cells, endothelial cells, or others, and contains membrane receptors as well as other proteins characteristic of the parental cell. Microparticles are heterogeneous in size, and are characterized as microvesicles free of nucleic acids. Also known as: cell membrane microparticle Subtypes: endothelial microparticle [GO:0072563] References: PMID:16373184 Sources: GOC:BHF, GOC:mah Relationships: is a type of cellular anatomical structure [GO:0110165]; is part of extracellular space [GO:0005615]